{
  "gene": "UniProtKB:Q9BVT8",
  "gene_symbol": "TMUB1",
  "term_id": "UNKNOWN:0003",
  "term_label": "Unknown cellular component",
  "gene_name": "Transmembrane and ubiquitin-like domain-containing protein 1"
}